{
  "gene_symbol": "NR0B1",
  "term_label": "male gonad development",
  "gene_name": "Nuclear receptor subfamily 0 group B member 1",
  "term_id": "GO:0008584",
  "gene": "UniProtKB:P51843"
}